volume-sensitive chloride channel activity [GO:0072320] (molecular function) Definition: Enables the transmembrane transfer of a chloride ion by a volume-sensitive channel. A volume-sensitive channel is a channel that responds to changes in the volume of a cell. Sources: GOC:mah Also known as: swell-activated chloride channel Relationships: is a type of volume-sensitive anion channel activity [GO:0005225]; is a type of chloride channel activity [GO:0005254]